{
  "gene": "UniProtKB:P15391",
  "gene_name": "B-lymphocyte antigen CD19",
  "gene_symbol": "CD19",
  "term_id": "UNKNOWN:0001",
  "term_label": "Unknown molecular function"
}